{
  "term_label": "SCF-dependent proteasomal ubiquitin-dependent protein catabolic process",
  "term_id": "GO:0031146",
  "gene_name": "F-box_LRR-repeat protein 2",
  "gene": "UniProtKB:Q9UKC9",
  "gene_symbol": "FBXL2"
}